protein localization to microvillus membrane [GO:1904107] (biological process) References: PMID:25335890 Sources: GOC:TermGenie, GOC:kmv, GO_REF:0000087 Definition: A process in which a protein is transported to, or maintained in, a location within a microvillus membrane. Also known as: protein localisation in microvillus membrane, protein localisation to microvillus membrane, protein localization in microvillus membrane Relationships: is a type of protein localization to membrane [GO:0072657]; is a type of protein localization to microvillus [GO:1904106]; is a type of protein localization to cell periphery [GO:1990778]